{
  "gene": "UniProtKB:Q9BVM2",
  "term_label": "Unknown biological process",
  "term_id": "UNKNOWN:0002",
  "gene_symbol": "DPCD",
  "gene_name": "Protein DPCD"
}